immune response in Peyer's patch [GO:0002388] (biological process) Sources: GOC:jal, ISBN:0781735149 Relationships: is a type of immune response in gut-associated lymphoid tissue [GO:0002387] Definition: Immune response taking place in the Peyer's patch, nodular lymphoid structures on the serosal surface of the small intestine. Subtypes: tolerance induction in Peyer's patch [GO:0002389]